{
  "gene_symbol": "MOBP",
  "gene_name": "Myelin-associated oligodendrocyte basic protein",
  "term_id": "UNKNOWN:0002",
  "gene": "UniProtKB:Q13875",
  "term_label": "Unknown biological process"
}